phosphatidylinositol-3,4,5-trisphosphate binding [GO:0005547] (molecular function) Definition: Binding to phosphatidylinositol-3,4,5-trisphosphate, a derivative of phosphatidylinositol in which the inositol ring is phosphorylated at the 3', 4' and 5' positions. Also known as: PIP3 binding Relationships: is a type of GO:0043168; is a type of GO:1901981 Sources: GOC:bf, GOC:jl